{
  "gene": "UniProtKB:Q14695",
  "term_label": "Unknown biological process",
  "term_id": "UNKNOWN:0002",
  "gene_name": "Uncharacterized protein KIAA0087",
  "gene_symbol": "KIAA0087"
}